negative regulation of phospholipid biosynthetic process [GO:0071072] (biological process) Definition: Any process that stops, prevents, or reduces the frequency, rate or extent of the chemical reactions and pathways resulting in the formation of phospholipids. Sources: GOC:mah Also known as: down regulation of phospholipid biosynthetic process, down-regulation of phospholipid biosynthetic process, downregulation of phospholipid biosynthetic process, negative regulation of phospholipid anabolism, negative regulation of phospholipid biosynthesis, negative regulation of phospholipid formation, negative regulation of phospholipid synthesis, inhibition of phospholipid biosynthetic process Relationships: is a type of GO:0051055; is_a regulation of phospholipid biosynthetic process [GO:0071071]; is_a negative regulation of phospholipid metabolic process [GO:1903726]; negatively regulates phospholipid biosynthetic process [GO:0008654] Subtypes: GO:0010323, negative regulation of phosphatidylinositol biosynthetic process [GO:0010512], GO:1900469, GO:1901352, negative regulation of phosphatidic acid biosynthetic process [GO:1905694], GO:2001211, GO:2001246